{
  "term_id": "GO:0008284",
  "term_label": "positive regulation of cell population proliferation",
  "gene_symbol": "OSMR",
  "gene_name": "Oncostatin-M-specific receptor subunit beta",
  "gene": "UniProtKB:Q99650"
}